{
  "gene_symbol": "FEV",
  "gene_name": "Protein FEV",
  "term_id": "GO:0000981",
  "term_label": "DNA-binding transcription factor activity, RNA polymerase II-specific",
  "gene": "UniProtKB:Q99581"
}